positive regulation of natural killer cell activation [GO:0032816] (biological process) Subtypes: positive regulation of natural killer cell proliferation [GO:0032819], GO:0032825 Also known as: positive regulation of NK cell activation, up regulation of natural killer cell activation, up-regulation of natural killer cell activation, upregulation of natural killer cell activation, activation of natural killer cell activation, stimulation of natural killer cell activation Definition: Any process that activates or increases the frequency, rate or extent of natural killer cell activation. Relationships: is a type of regulation of natural killer cell activation [GO:0032814]; is a type of positive regulation of lymphocyte activation [GO:0051251]; positively regulates natural killer cell activation [GO:0030101] Sources: GOC:mah